{
  "term_label": "calcium ion import across plasma membrane",
  "gene_name": "Transient receptor potential cation channel subfamily V member 5",
  "gene": "UniProtKB:Q9NQA5",
  "gene_symbol": "TRPV5",
  "term_id": "GO:0098703"
}